{
  "gene": "UniProtKB:Q86V71",
  "gene_name": "Zinc finger protein 429",
  "term_label": "RNA polymerase II cis-regulatory region sequence-specific DNA binding",
  "gene_symbol": "ZNF429",
  "term_id": "GO:0000978"
}